{
  "term_id": "GO:0031267",
  "gene_name": "MICAL-like protein 1",
  "gene": "UniProtKB:Q8N3F8",
  "gene_symbol": "MICALL1",
  "term_label": "small GTPase binding"
}